{
  "term_label": "neuromuscular synaptic transmission",
  "term_id": "GO:0007274",
  "gene_symbol": "CHRNA3",
  "gene_name": "Neuronal acetylcholine receptor subunit alpha-3",
  "gene": "UniProtKB:P32297"
}